{
  "term_id": "UNKNOWN:0002",
  "gene_name": "Endogenous retrovirus group FC1 Env polyprotein",
  "gene": "UniProtKB:P60507",
  "term_label": "Unknown biological process",
  "gene_symbol": "ERVFC1"
}